regulation of glial cell proliferation [GO:0060251] (biological process) Relationships: is a type of GO:0042127; regulates glial cell proliferation [GO:0014009] Definition: Any process that modulates the frequency, rate or extent of glial cell proliferation. Sources: GOC:dph, GOC:tb Subtypes: regulation of Schwann cell proliferation [GO:0010624], GO:0060252, negative regulation of glial cell proliferation [GO:0060253]